{
  "gene": "UniProtKB:Q9Y3C8",
  "term_label": "cytoplasm",
  "term_id": "GO:0005737",
  "gene_symbol": "UFC1",
  "gene_name": "Ubiquitin-fold modifier-conjugating enzyme 1"
}